{
  "gene_symbol": "SLC1A1",
  "gene": "UniProtKB:P43005",
  "gene_name": "Excitatory amino acid transporter 3",
  "term_id": "GO:0033229",
  "term_label": "cysteine transmembrane transporter activity"
}